lipid droplet formation [GO:0140042] (biological process) Definition: A process that results in the assembly, arrangement of constituent parts of a lipid droplet. References: PMID:28011631 Also known as: adiposome formation, lipid body formation, lipid particle formation Relationships: is a type of GO:0034389; is a type of membraneless organelle assembly [GO:0140694]; is part of lipid storage [GO:0019915]